{
  "term_label": "mitochondrion organization",
  "gene_symbol": "MSTO1",
  "term_id": "GO:0007005",
  "gene_name": "Protein misato homolog 1",
  "gene": "UniProtKB:Q9BUK6"
}